lens fiber cell apoptotic process [GO:1990086] (biological process) Relationships: is a type of GO:1904019 Definition: Any apoptotic process in a lens fiber cell. Lens fiber cells are elongated, tightly packed cells that make up the bulk of the mature lens in a camera-type eye. References: PMID:11095619 Sources: CL:0011004, GOC:hjd